beta-L-Ara4N-lipid A biosynthetic process [GO:1901760] (BP) Also known as: 4-amino-4-deoxy-beta-L-arabinose-lipid A biosynthesis, 4-amino-4-deoxy-beta-L-arabinose-lipid A biosynthetic process, beta-L-Ara4N-lipid A anabolism, beta-L-Ara4N-lipid A biosynthesis, beta-L-Ara4N-lipid A formation, beta-L-Ara4N-lipid A synthesis Definition: The chemical reactions and pathways resulting in the formation of beta-L-Ara4N-lipid A which occurs as a result of modification of the lipid A moiety of lipopolysaccharide by the addition of the sugar 4-amino-4-deoxy-L-arabinose (L-Ara4N). This strategy is adopted by pathogenic Gram-negative bacteria to evade cationic antimicrobial peptides produced by the innate immune system. Relationships: is a type of phospholipid biosynthetic process [GO:0008654]; is_a glycolipid biosynthetic process [GO:0009247]; is a type of GO:1901271 References: PMID:17928292, PMID:19166326 Sources: GOC:TermGenie, GOC:yaf, UniPathway:UPA00037